(4S)-4-hydroxy-2-oxoglutarate aldolase activity [GO:0106009] (molecular function) Relationships: is a type of oxo-acid-lyase activity [GO:0016833] References: PMID:1098660, PMID:1339418 Sources: RHEA:35639 Definition: Catalysis of the reaction:(4S)-4-hydroxy-2-oxoglutarate = pyruvate + glyoxylate. Specific for the (4S) enantiomer of 4-hydroxy-2-oxoglutarate.